{
  "term_label": "Unknown biological process",
  "gene": "UniProtKB:Q68CJ6",
  "gene_name": "Nuclear GTPase SLIP-GC",
  "gene_symbol": "NUGGC",
  "term_id": "UNKNOWN:0002"
}